{
  "gene": "UniProtKB:Q9Y2T3",
  "term_label": "cytosol",
  "gene_name": "Guanine deaminase",
  "term_id": "GO:0005829",
  "gene_symbol": "GDA"
}